cellular response to linoleic acid [GO:0071399] (biological process) Definition: Any process that results in a change in state or activity of a cell (in terms of movement, secretion, enzyme production, gene expression, etc.) as a result of a linoleic acid stimulus. Sources: GOC:mah Relationships: is a type of response to linoleic acid [GO:0070543]; is a type of cellular response to fatty acid [GO:0071398] Also known as: cellular response to linoleate